{
  "term_label": "Unknown biological process",
  "gene_symbol": "NDUFAB1",
  "term_id": "UNKNOWN:0002",
  "gene_name": "Acyl carrier protein, mitochondrial",
  "gene": "UniProtKB:O14561"
}